viral outer capsid [GO:0039624] (cellular component) Definition: The outer layer of a double or triple concentric icosahedral capsid. Outer capsids are part of reoviridae and cystoviridae virions. Also known as: outer capsid Relationships: is a type of virion component [GO:0044423]; BFO_0000050 GO:0019030 Sources: UniProtKB-KW:KW-1152